{
  "term_label": "NLRP3 inflammasome complex",
  "gene": "UniProtKB:Q9Y2G2",
  "gene_symbol": "CARD8",
  "gene_name": "Caspase recruitment domain-containing protein 8",
  "term_id": "GO:0072559"
}